{
  "term_label": "late endosome to Golgi transport",
  "gene_symbol": "SNX3",
  "gene_name": "Sorting nexin-3",
  "term_id": "GO:0034499",
  "gene": "UniProtKB:O60493"
}